hyphal tip [GO:0001411] (cellular component) Relationships: is a type of GO:0030427; is a type of cell tip [GO:0051286] Sources: GOC:mcc Definition: The end, or tip, of a fungal hypha, where polarized growth occurs during hyphal elongation.